{
  "term_label": "spliceosomal complex",
  "gene_symbol": "CIRBP",
  "term_id": "GO:0005681",
  "gene": "UniProtKB:Q14011",
  "gene_name": "Cold-inducible RNA-binding protein"
}